{
  "gene_symbol": "ZFYVE1",
  "term_label": "1-phosphatidylinositol binding",
  "term_id": "GO:0005545",
  "gene_name": "Zinc finger FYVE domain-containing protein 1",
  "gene": "UniProtKB:Q9HBF4"
}